{
  "gene_symbol": "RPUSD1",
  "term_id": "UNKNOWN:0003",
  "gene": "UniProtKB:Q9UJJ7",
  "gene_name": "RNA pseudouridylate synthase domain-containing protein 1",
  "term_label": "Unknown cellular component"
}